{
  "gene": "UniProtKB:Q8NBR0",
  "term_label": "cytoplasm",
  "gene_symbol": "TP53I13",
  "gene_name": "Tumor protein p53-inducible protein 13",
  "term_id": "GO:0005737"
}